fusiform vesicle [GO:0120002] (cellular component) Definition: A cytoplasmic vesicle which contains two urothelial plaques and can deliver these plaques to the apical plasma membrane of urothelial superficial (umbrella) cells. It can also be formed by endocytosis of apical plasma membrane during contractions of the urinary bladder. Relationships: is a type of cytoplasmic vesicle [GO:0031410] References: PMID:21468280, PMID:21887288 Sources: GOC:krc